{
  "gene_name": "Ran-binding protein 10",
  "gene": "UniProtKB:Q6VN20",
  "term_id": "GO:0030674",
  "gene_symbol": "RANBP10",
  "term_label": "protein-macromolecule adaptor activity"
}